plant seed peroxygenase activity [GO:1990137] (molecular function) Definition: Catalysis of the reaction: RH + ROOH = ROH + ROH. References: PMID:19467604 Sources: EC:1.11.2.3 Also known as: peroxygenase activity, plant seed peroxidase activity Relationships: is_a oxidoreductase activity, acting on peroxide as acceptor [GO:0016684]